{
  "gene": "UniProtKB:Q96GS4",
  "gene_name": "BLOC-1-related complex subunit 6",
  "term_label": "BORC complex",
  "term_id": "GO:0099078",
  "gene_symbol": "BORCS6"
}